{
  "gene_name": "GTP-binding protein Di-Ras3",
  "gene": "UniProtKB:O95661",
  "gene_symbol": "DIRAS3",
  "term_id": "GO:0005886",
  "term_label": "plasma membrane"
}